{
  "gene_symbol": "GOSR2",
  "term_label": "SNAP receptor activity",
  "gene": "UniProtKB:O14653",
  "gene_name": "Golgi SNAP receptor complex member 2",
  "term_id": "GO:0005484"
}